{
  "term_label": "lipopolysaccharide-mediated signaling pathway",
  "gene": "UniProtKB:O43187",
  "term_id": "GO:0031663",
  "gene_symbol": "IRAK2",
  "gene_name": "Interleukin-1 receptor-associated kinase-like 2"
}